{
  "term_id": "GO:0000254",
  "gene": "UniProtKB:Q96IV6",
  "term_label": "C-4 methylsterol oxidase activity",
  "gene_symbol": "FAXDC2",
  "gene_name": "Fatty acid hydroxylase domain-containing protein 2"
}